N-(4-hydroxybenzoyl)-L-glutamate synthetase activity [GO:0052628] (molecular function) Also known as: 4-hydroxybenzoate amino acid synthetase activity, 4-hydroxybenzoyl amino acid synthetase activity, 4HBA amino acid synthetase activity, p-hydroxybenzoate amino acid synthetase activity, p-hydroxybenzoyl amino acid synthetase activity Relationships: is a type of GO:0016881 Definition: Catalysis of the reaction: 4-hydroxybenzoate + L-glutamate + ATP = N-(4-hydroxybenzoyl)-L-glutamate + AMP + diphosphate + H+. References: PMID:19189963 Sources: MetaCyc:RXN-10887